{
  "term_label": "Unknown cellular component",
  "term_id": "UNKNOWN:0003",
  "gene_symbol": "TYMSOS",
  "gene": "UniProtKB:Q8TAI1",
  "gene_name": "TYMS opposite strand protein"
}